{
  "gene_symbol": "BBS7",
  "gene": "UniProtKB:Q8IWZ6",
  "term_label": "Unknown molecular function",
  "term_id": "UNKNOWN:0001",
  "gene_name": "Bardet-Biedl syndrome 7 protein"
}